{
  "gene_symbol": "SMYD1",
  "term_id": "GO:0007507",
  "term_label": "heart development",
  "gene": "UniProtKB:Q8NB12",
  "gene_name": "Histone-lysine N-methyltransferase SMYD1"
}